{
  "term_id": "UNKNOWN:0003",
  "gene_name": "Interleukin enhancer-binding factor 2",
  "gene_symbol": "ILF2",
  "term_label": "Unknown cellular component",
  "gene": "UniProtKB:Q12905"
}